{
  "gene_symbol": "SYT4",
  "gene": "UniProtKB:Q9H2B2",
  "term_id": "GO:0016192",
  "term_label": "vesicle-mediated transport",
  "gene_name": "Synaptotagmin-4"
}